{
  "gene_name": "Mid1-interacting protein 1",
  "gene_symbol": "MID1IP1",
  "gene": "UniProtKB:Q9NPA3",
  "term_id": "GO:0005829",
  "term_label": "cytosol"
}